{
  "gene": "UniProtKB:Q3KNT7",
  "gene_name": "Putative NOL1_NOP2_Sun domain family member 5B",
  "term_id": "UNKNOWN:0003",
  "term_label": "Unknown cellular component",
  "gene_symbol": "NSUN5P1"
}